{
  "gene": "UniProtKB:A6NHT5",
  "gene_name": "Homeobox protein HMX3",
  "gene_symbol": "HMX3",
  "term_label": "nucleus",
  "term_id": "GO:0005634"
}